{
  "gene": "UniProtKB:Q9Y5Z9",
  "term_id": "GO:0042371",
  "gene_name": "UbiA prenyltransferase domain-containing protein 1",
  "gene_symbol": "UBIAD1",
  "term_label": "vitamin K biosynthetic process"
}